{
  "term_id": "GO:0000400",
  "term_label": "four-way junction DNA binding",
  "gene": "UniProtKB:Q17RS7",
  "gene_symbol": "GEN1",
  "gene_name": "Flap endonuclease GEN homolog 1"
}